{
  "term_label": "cytoskeleton-dependent cytokinesis",
  "gene_name": "Septin-7",
  "term_id": "GO:0061640",
  "gene": "UniProtKB:Q16181",
  "gene_symbol": "SEPTIN7"
}